{
  "term_id": "GO:0004693",
  "gene": "UniProtKB:Q96Q40",
  "gene_symbol": "CDK15",
  "gene_name": "Cyclin-dependent kinase 15",
  "term_label": "cyclin-dependent protein serine/threonine kinase activity"
}